{
  "term_label": "Golgi apparatus",
  "gene": "UniProtKB:Q9Y6M5",
  "gene_symbol": "SLC30A1",
  "term_id": "GO:0005794",
  "gene_name": "Proton-coupled zinc antiporter SLC30A1"
}